{
  "gene_name": "Immunoglobulin heavy variable 3-33",
  "gene": "UniProtKB:P01772",
  "term_label": "Unknown cellular component",
  "term_id": "UNKNOWN:0003",
  "gene_symbol": "IGHV3-33"
}